{
  "term_label": "ubiquitin conjugating enzyme binding",
  "gene_name": "E3 ubiquitin-protein ligase RNF144A",
  "gene": "UniProtKB:P50876",
  "gene_symbol": "RNF144A",
  "term_id": "GO:0031624"
}